regulation of cardiac muscle cell action potential [GO:0098901] (biological process) Subtypes: GO:0098904, GO:0098905, regulation of Purkinje myocyte action potential [GO:0098906], GO:0098907, regulation of cardiac muscle cell action potential involved in regulation of contraction [GO:0098909], regulation of atrial cardiac muscle cell action potential [GO:0098910], regulation of ventricular cardiac muscle cell action potential [GO:0098911] Sources: GOC:dos, GOC:mtg_cardiac_conduct_nov11 Relationships: is a type of GO:0098900; regulates cardiac muscle cell action potential [GO:0086001] Definition: Any process that modulates the frequency, rate or extent of action potential creation, propagation or termination in a cardiac muscle cell. This typically occurs via modulation of the activity or expression of voltage-gated ion channels.